{
  "term_label": "cytoplasm",
  "gene": "UniProtKB:Q15102",
  "gene_symbol": "PAFAH1B3",
  "gene_name": "Platelet-activating factor acetylhydrolase IB subunit alpha1",
  "term_id": "GO:0005737"
}